{
  "term_id": "GO:0005737",
  "gene_name": "Peptidyl-prolyl cis-trans isomerase A-like 4G",
  "gene_symbol": "PPIAL4G",
  "term_label": "cytoplasm",
  "gene": "UniProtKB:P0DN37"
}